{
  "gene": "UniProtKB:Q96P64",
  "gene_symbol": "AGAP4",
  "term_label": "Unknown biological process",
  "gene_name": "Arf-GAP with GTPase, ANK repeat and PH domain-containing protein 4",
  "term_id": "UNKNOWN:0002"
}